{
  "term_label": "nerve growth factor signaling pathway",
  "term_id": "GO:0038180",
  "gene_symbol": "BDNF",
  "gene": "UniProtKB:P23560",
  "gene_name": "Brain-derived neurotrophic factor"
}